{
  "term_label": "Unknown cellular component",
  "gene": "UniProtKB:Q5VTM2",
  "term_id": "UNKNOWN:0003",
  "gene_name": "Arf-GAP with GTPase, ANK repeat and PH domain-containing protein 9",
  "gene_symbol": "AGAP9"
}